{
  "gene_symbol": "EDDM3A",
  "term_id": "UNKNOWN:0003",
  "gene": "UniProtKB:Q14507",
  "gene_name": "Epididymal secretory protein E3-alpha",
  "term_label": "Unknown cellular component"
}